{
  "gene_symbol": "TXNL4A",
  "term_label": "U5 snRNP",
  "gene_name": "Thioredoxin-like protein 4A",
  "gene": "UniProtKB:P83876",
  "term_id": "GO:0005682"
}